{
  "term_id": "GO:0006420",
  "gene": "UniProtKB:Q5T160",
  "gene_symbol": "RARS2",
  "term_label": "arginyl-tRNA aminoacylation",
  "gene_name": "Probable arginine--tRNA ligase, mitochondrial"
}